{
  "gene_name": "Glycine receptor subunit alpha-1",
  "gene": "UniProtKB:P23415",
  "gene_symbol": "GLRA1",
  "term_id": "UNKNOWN:0003",
  "term_label": "Unknown cellular component"
}